{
  "gene_symbol": "CACNA1C",
  "gene": "UniProtKB:Q13936",
  "term_id": "GO:0008331",
  "gene_name": "Voltage-dependent L-type calcium channel subunit alpha-1C",
  "term_label": "high voltage-gated calcium channel activity"
}